{
  "gene_symbol": "MAGED2",
  "gene": "UniProtKB:Q9UNF1",
  "term_label": "Unknown molecular function",
  "gene_name": "Melanoma-associated antigen D2",
  "term_id": "UNKNOWN:0001"
}